{
  "term_label": "nucleus",
  "gene": "UniProtKB:Q9BXY8",
  "gene_symbol": "BEX2",
  "term_id": "GO:0005634",
  "gene_name": "Protein BEX2"
}